{
  "gene_symbol": "NTM-AS1",
  "term_label": "Unknown biological process",
  "term_id": "UNKNOWN:0002",
  "gene_name": "Putative uncharacterized protein NTM-AS1",
  "gene": "UniProtKB:Q6ZSK4"
}